negative regulation of isotype switching to IgA isotypes [GO:0048297] (biological process) Also known as: down regulation of isotype switching to IgA isotypes, down-regulation of isotype switching to IgA isotypes, downregulation of isotype switching to IgA isotypes, negative regulation of class switch recombination to IgA isotypes, negative regulation of class switching to IgA isotypes, negative regulation of isotype switch recombination to IgA isotypes, inhibition of isotype switching to IgA isotypes Definition: Any process that stops, prevents, or reduces the frequency, rate or extent of isotype switching to IgA isotypes. Relationships: is a type of negative regulation of isotype switching [GO:0045829]; is a type of GO:0048296; negatively regulates isotype switching to IgA isotypes [GO:0048290] Sources: GOC:jid